{
  "gene_name": "TBC1 domain family member 10A",
  "gene": "UniProtKB:Q9BXI6",
  "term_label": "retrograde transport, endosome to Golgi",
  "term_id": "GO:0042147",
  "gene_symbol": "TBC1D10A"
}